{
  "gene": "UniProtKB:Q5W5X9",
  "term_label": "Unknown molecular function",
  "term_id": "UNKNOWN:0001",
  "gene_symbol": "TTC23",
  "gene_name": "Tetratricopeptide repeat protein 23"
}